3-hydroxypropionyl-CoA synthetase activity [GO:0043955] (molecular function) Also known as: AMP-dependent synthetase and ligase, AMP-dependent synthetase and ligase:Enoyl-CoA hydratase/isomerase, acetyl-coenzyme A synthetase, enoyl-CoA hydratase/isomerase, 3-hydroxy propionyl-CoA synthetase activity, acetyl-coenzyme A synthetase/GroES-like domain Relationships: is a type of GO:0016405; is a type of acid-thiol ligase activity [GO:0016878] Definition: Catalysis of the reaction: 3-hydroxypropionate + ATP + CoA = 3-hydroxypropionyl-CoA + AMP + diphosphate. References: PMID:11821399 Sources: GOC:jl Note: Note that this function is one of the activities of the trifunctional enzyme propionyl-coenzyme A synthase. See PMID:11821399.